{
  "gene": "UniProtKB:A0A0C4DH34",
  "term_label": "antigen binding",
  "term_id": "GO:0003823",
  "gene_name": "Immunoglobulin heavy variable 4-28",
  "gene_symbol": "IGHV4-28"
}